{
  "gene_symbol": "PET117",
  "gene_name": "Protein PET117 homolog, mitochondrial",
  "term_id": "GO:0005739",
  "gene": "UniProtKB:Q6UWS5",
  "term_label": "mitochondrion"
}